intermediate filament cytoskeleton [GO:0045111] (cellular component) Sources: ISBN:0716731363 Subtypes: neurofilament cytoskeleton [GO:0060053], postsynaptic intermediate filament cytoskeleton [GO:0099160], presynaptic intermediate filament cytoskeleton [GO:0099182] Definition: Cytoskeletal structure made from intermediate filaments, typically organized in the cytosol as an extended system that stretches from the nuclear envelope to the plasma membrane. Some intermediate filaments run parallel to the cell surface, while others traverse the cytosol; together they form an internal framework that helps support the shape and resilience of the cell. Relationships: is a type of cytoskeleton [GO:0005856]